{
  "gene": "UniProtKB:Q6N022",
  "gene_symbol": "TENM4",
  "term_id": "GO:0046982",
  "gene_name": "Teneurin-4",
  "term_label": "protein heterodimerization activity"
}